dinoflagellate peduncle [GO:1990905] (cellular component) Note: The term name refers to a taxonomic group to make the label unique with respect to similarly-named anatomical structures. Definition: A small, flexible, finger-like projection of cytoplasm containing an array of microtubles and located near the flagellar pores in some photosynthetic as well as nonphotosynthetic dinoflagellate species. Its functions are not fully understood, but it has been associated with feeding behavior (phagotrophy). Relationships: is a type of plasma membrane bounded cell projection [GO:0120025] References: PMID:1480107 Sources: GOC:at, Wikipedia:Dinoflagellate